diphthine methylesterase activity [GO:0061685] (molecular function) Relationships: is a type of carboxylic ester hydrolase activity [GO:0052689] References: PMID:24739148 Sources: GOC:dph, RHEA:42656 Definition: Catalysis of the reaction: diphthine methyl ester + H2O = diphthine + H+ + methanol.